protein transport along microtubule to spindle pole body [GO:1990852] (biological process) Definition: The directed movement of a protein along a microtubule to the spindle pole body, mediated by motor proteins. Subtypes: protein transport along microtubule to mitotic spindle pole body [GO:1990976] Relationships: is a type of GO:0071989; is a type of protein transport along microtubule [GO:0098840] References: PMID:25987607